{
  "gene_name": "Laminin subunit gamma-3",
  "gene_symbol": "LAMC3",
  "term_id": "GO:0005604",
  "gene": "UniProtKB:Q9Y6N6",
  "term_label": "basement membrane"
}